{
  "term_label": "autophagosome assembly",
  "gene": "UniProtKB:Q96BY7",
  "gene_symbol": "ATG2B",
  "gene_name": "Autophagy-related protein 2 homolog B",
  "term_id": "GO:0000045"
}